ent-kaurene metabolic process [GO:0033331] (biological process) References: PMID:17064690 Sources: GOC:mah Also known as: ent-kaurene metabolism Subtypes: ent-kaurene oxidation to kaurenoic acid [GO:0010241], ent-kaurene biosynthetic process [GO:0033332] Relationships: is a type of GO:0042214 Definition: The chemical reactions and pathways involving ent-kaur-16-ene. Ent-kaurene is a tetracyclic diterpenoid that is a precursor of several plant isoprenoids, including gibberellins.